{
  "gene_symbol": "RWDD1",
  "term_id": "GO:0002181",
  "gene_name": "RWD domain-containing protein 1",
  "term_label": "cytoplasmic translation",
  "gene": "UniProtKB:Q9H446"
}